dopachrome isomerase activity [GO:0004167] (molecular function) Relationships: is_a intramolecular oxidoreductase activity, transposing C=C bonds [GO:0016863] Definition: Catalysis of the reaction: L-dopachrome = 5,6-dihydroxyindole-2-carboxylate. Also known as: dopachrome conversion activity, dopachrome conversion factor activity, dopachrome delta-isomerase activity, DCF activity, DCT activity, L-dopachrome isomerase activity, L-dopachrome keto-enol isomerase activity, L-dopachrome-methyl ester tautomerase activity, TRP activity, TRP-1, TRP-2, TRP2, dopachrome Delta(7),Delta(2)-isomerase activity, dopachrome delta7,Delta2-isomerase activity, dopachrome keto-enol isomerase activity, dopachrome oxidoreductase activity, dopachrome rearranging enzyme activity, dopachrome tautomerase activity, dopachrome-rearranging enzyme, tryosinase-related protein-2, tyrosinase-related protein 2 activity Sources: EC:5.3.3.12, RHEA:13041